{
  "term_id": "GO:0005789",
  "gene_name": "cTAGE family member 4",
  "gene_symbol": "CTAGE4",
  "term_label": "endoplasmic reticulum membrane",
  "gene": "UniProtKB:Q8IX94"
}